{
  "term_id": "GO:0004364",
  "term_label": "glutathione transferase activity",
  "gene_name": "Maleylacetoacetate isomerase",
  "gene": "UniProtKB:O43708",
  "gene_symbol": "GSTZ1"
}